{
  "gene": "UniProtKB:A5A3E0",
  "term_label": "cytoplasm",
  "gene_symbol": "POTEF",
  "gene_name": "POTE ankyrin domain family member F",
  "term_id": "GO:0005737"
}